{
  "term_label": "uracil DNA N-glycosylase activity",
  "gene_name": "Uracil-DNA glycosylase",
  "gene": "UniProtKB:P13051",
  "gene_symbol": "UNG",
  "term_id": "GO:0004844"
}